regulation of glomerular filtration [GO:0003093] (biological process) Sources: GOC:mtg_cardio Definition: Any process that modulates the frequency, rate or extent of glomerular filtration. Glomerular filtration is the process in which blood is filtered by the glomerulus into the renal tubule. Subtypes: GO:0003104, negative regulation of glomerular filtration [GO:0003105] Relationships: is a type of GO:0001977; is a type of regulation of renal system process [GO:0098801]; regulates glomerular filtration [GO:0003094]